endosome fission [GO:0140285] (biological process) References: PMID:25416943, PMID:30220460 Relationships: is a type of organelle fission [GO:0048285] Definition: The process by which early and late endosomes undergo budding and fission reactions that separate regions destined for lysosomal degradation from carriers to be recycled to the plasma membrane.